{
  "gene_name": "Activin receptor type-2A",
  "term_id": "GO:0032924",
  "gene": "UniProtKB:P27037",
  "gene_symbol": "ACVR2A",
  "term_label": "activin receptor signaling pathway"
}